columbamine O-methyltransferase activity [GO:0030778] (MF) Definition: Catalysis of the reaction: S-adenosyl-L-methionine + columbamine = S-adenosyl-L-homocysteine + H+ + palmatine. Relationships: is a type of GO:0008757 Also known as: S-adenosyl-L-methionine:columbamine O-methyltransferase activity Sources: EC:2.1.1.118, RHEA:15373